beta-glucan metabolic process [GO:0051273] (biological process) Definition: The chemical reactions and pathways involving beta-glucans, compounds composed of glucose residues linked by beta-D-glucosidic bonds. Relationships: is a type of glucan metabolic process [GO:0044042] Also known as: beta-glucan metabolism Regulation: RO_0002211 by regulation of beta-glucan metabolic process [GO:0032950] Subtypes: (1->3)-beta-D-glucan metabolic process [GO:0006074], (1->6)-beta-D-glucan metabolic process [GO:0006077], GO:0030243, cell wall beta-glucan metabolic process [GO:0034406], beta-glucan biosynthetic process [GO:0051274], GO:0051275 Sources: GOC:ai